{
  "gene_name": "Sperm protein associated with the nucleus on the X chromosome A",
  "term_id": "UNKNOWN:0002",
  "gene_symbol": "SPANXA2",
  "term_label": "Unknown biological process",
  "gene": "UniProtKB:Q9NS26"
}